{
  "gene": "UniProtKB:Q96HC4",
  "gene_name": "PDZ and LIM domain protein 5",
  "term_id": "GO:0001725",
  "gene_symbol": "PDLIM5",
  "term_label": "stress fiber"
}